nuclear pore outer ring [GO:0031080] (cellular component) Also known as: Nup107-120 complex, Nup107-160 complex, Nup84 complex Relationships: is a type of nuclear protein-containing complex [GO:0140513]; is part of nuclear pore [GO:0005643] References: PMID:18046406, PMID:19524430, PMID:20947011, PMID:22419078 Sources: GOC:dgf Definition: A subcomplex of the nuclear pore complex (NPC) that forms the outer rings of the core scaffold, a lattice-like structure that gives the NPC its shape and strength. In S. cerevisiae, the two outer rings each contain multiple copies of the following proteins: Nup133p, Nup120p, Nup145Cp, Nup85p, Nup84p, Seh1p, and Sec13p. In vertebrates, the two outer rings each contain multiple copies of the following proteins: Nup133, Nup160, Nup96, Nup75, Nup107, Seh1, Sec13, Nup43, Nup37, and ALADIN. Components are arranged in 8-fold symmetrical 'spokes' around the central transport channel. A single 'spoke', can be isolated and is sometimes referred to as the Nup84 complex (S. cerevisiae) or the Nup107-160 complex (vertebrates).